{
  "term_id": "GO:0007162",
  "term_label": "negative regulation of cell adhesion",
  "gene": "UniProtKB:P01042",
  "gene_name": "Kininogen-1",
  "gene_symbol": "KNG1"
}